{
  "gene_symbol": "ENTREP2",
  "term_label": "Unknown cellular component",
  "term_id": "UNKNOWN:0003",
  "gene_name": "Protein ENTREP2",
  "gene": "UniProtKB:O60320"
}